{
  "gene_symbol": "RAB9A",
  "term_id": "UNKNOWN:0001",
  "term_label": "Unknown molecular function",
  "gene": "UniProtKB:P51151",
  "gene_name": "Ras-related protein Rab-9A"
}